{
  "gene": "UniProtKB:P0DX00",
  "term_id": "UNKNOWN:0001",
  "term_label": "Unknown molecular function",
  "gene_symbol": "GOLGA6L24",
  "gene_name": "Golgin subfamily A member 6-like protein 24"
}